{
  "gene_symbol": "ECM2",
  "term_id": "GO:0008201",
  "term_label": "heparin binding",
  "gene": "UniProtKB:O94769",
  "gene_name": "Extracellular matrix protein 2"
}